cobalt-precorrin-6B C5-methyltransferase activity [GO:0043776] (molecular function) Sources: MetaCyc:RXN-8766 Also known as: precorrin-6Y C5,15-methyltransferase (decarboxylating), precorrin-6Y methylase, cobalt-precorrin 6B C5-methyltransferase activity, precorrin-6 methyltransferase activity Definition: Catalysis of the reaction: S-adenosylmethionine + cobalt-precorrin 6B = S-adenosylhomocysteine + cobalt-precorrin 7. Relationships: is a type of methyltransferase activity [GO:0008168]